positive regulation of circadian sleep/wake cycle, non-REM sleep [GO:0046010] (biological process) Relationships: is a type of regulation of circadian sleep/wake cycle, non-REM sleep [GO:0045188]; is a type of GO:0045938; positively regulates GO:0042748 Sources: GOC:go_curators Also known as: positive regulation of non-REM sleep, up regulation of circadian sleep/wake cycle, non-REM sleep, up-regulation of circadian sleep/wake cycle, non-REM sleep, upregulation of circadian sleep/wake cycle, non-REM sleep, activation of circadian sleep/wake cycle, non-REM sleep, stimulation of circadian sleep/wake cycle, non-REM sleep Definition: Any process that activates or increases the duration or quality of non-rapid eye movement (NREM) sleep.